{
  "gene_symbol": "FUT8",
  "term_label": "alpha-(1->6)-fucosyltransferase activity",
  "gene": "UniProtKB:Q9BYC5",
  "gene_name": "Alpha-(1,6)-fucosyltransferase",
  "term_id": "GO:0046921"
}